{
  "term_label": "central nervous system development",
  "gene_symbol": "DSCAM",
  "gene_name": "Cell adhesion molecule DSCAM",
  "term_id": "GO:0007417",
  "gene": "UniProtKB:O60469"
}